{
  "gene_name": "Mas-related G-protein coupled receptor MRG",
  "gene_symbol": "MAS1L",
  "gene": "UniProtKB:P35410",
  "term_id": "GO:0004930",
  "term_label": "G protein-coupled receptor activity"
}